{
  "gene_symbol": "TENM2",
  "term_label": "cell adhesion molecule binding",
  "gene_name": "Teneurin-2",
  "term_id": "GO:0050839",
  "gene": "UniProtKB:Q9NT68"
}